{
  "gene": "UniProtKB:Q8N1W1",
  "term_id": "UNKNOWN:0003",
  "gene_name": "Rho guanine nucleotide exchange factor 28",
  "gene_symbol": "ARHGEF28",
  "term_label": "Unknown cellular component"
}